{
  "gene": "UniProtKB:Q8NH16",
  "gene_name": "Olfactory receptor 2L2",
  "gene_symbol": "OR2L2",
  "term_id": "GO:0004984",
  "term_label": "olfactory receptor activity"
}